actin severing activator activity [GO:0000513] (molecular function) References: PMID:25451933 Relationships: is a type of GO:0140677 Definition: Binds to and increases the activity of a actin severing protein.